{
  "term_id": "GO:0005525",
  "term_label": "GTP binding",
  "gene_symbol": "DRG1",
  "gene": "UniProtKB:Q9Y295",
  "gene_name": "Developmentally-regulated GTP-binding protein 1"
}